{
  "gene_name": "F-box_WD repeat-containing protein 11",
  "term_label": "microtubule plus-end binding",
  "term_id": "GO:0051010",
  "gene": "UniProtKB:Q9UKB1",
  "gene_symbol": "FBXW11"
}